{
  "gene_symbol": "FAM90A16",
  "gene_name": "Protein FAM90A16",
  "term_id": "UNKNOWN:0003",
  "gene": "UniProtKB:P0DV73",
  "term_label": "Unknown cellular component"
}